positive regulation of interleukin-11 production [GO:0032734] (biological process) Also known as: positive regulation of IL-11 production, up regulation of interleukin-11 production, up-regulation of interleukin-11 production, upregulation of interleukin-11 production, activation of interleukin-11 production, positive regulation of interleukin-11 biosynthetic process, positive regulation of interleukin-11 secretion, stimulation of interleukin-11 production Relationships: is a type of positive regulation of cytokine production [GO:0001819]; is a type of GO:0032654; positively regulates interleukin-11 production [GO:0032614] Sources: GOC:mah Definition: Any process that activates or increases the frequency, rate, or extent of interleukin-11 production.